{
  "gene_name": "Connector enhancer of kinase suppressor of ras 1",
  "gene": "UniProtKB:Q969H4",
  "term_id": "UNKNOWN:0003",
  "gene_symbol": "CNKSR1",
  "term_label": "Unknown cellular component"
}